biofilm formation [GO:0042710] (biological process) References: PMID:11932229 Sources: GOC:di Subtypes: single-species biofilm formation [GO:0044010], multi-species biofilm formation [GO:0044399], surface biofilm formation [GO:0090604], submerged biofilm formation [GO:0090605] Relationships: is a type of aggregation of unicellular organisms [GO:0098630] Definition: A process in which planktonically growing microorganisms grow at a liquid-air interface or on a solid substrate under the flow of a liquid and produce extracellular polymers that facilitate matrix formation, resulting in a change in the organisms' growth rate and gene transcription.